{
  "term_id": "GO:0044183",
  "gene_symbol": "DNAJB7",
  "gene_name": "DnaJ homolog subfamily B member 7",
  "gene": "UniProtKB:Q7Z6W7",
  "term_label": "protein folding chaperone"
}